{
  "gene": "UniProtKB:P09467",
  "term_label": "cytosol",
  "term_id": "GO:0005829",
  "gene_name": "Fructose-1,6-bisphosphatase 1",
  "gene_symbol": "FBP1"
}